extracellular exosome biogenesis [GO:0097734] (biological process) Relationships: is a type of extracellular vesicle biogenesis [GO:0140112] Definition: The assembly and secretion of an extracellular exosome, a membrane-bounded vesicle that is released into the extracellular region by fusion of the limiting endosomal membrane of a multivesicular body with the plasma membrane. References: PMID:19442504, PMID:25392495 Sources: GOC:PARL, GOC:bf Also known as: exosome assembly or secretion, exosome biogenesis, exosome production, ILV assembly, intraluminal vesicle assembly